CDP-diacylglycerol-serine O-phosphatidyltransferase activity [GO:0003882] (molecular function) Sources: EC:2.7.8.8 Definition: Catalysis of the reaction: CDP-diacylglycerol + L-serine = CMP + O-sn-phosphatidyl-L-serine. Relationships: is_a GO:0017169 Also known as: serine exchange enzyme, CDP-diacylglycerol-L-serine O-phosphatidyltransferase activity, CDP-diacylglycerol:L-serine 3-O-phosphatidyltransferase activity, CDP-diglyceride-L-serine phosphatidyltransferase activity, CDP-diglyceride:serine phosphatidyltransferase activity, CDP-diglycerine-serine O-phosphatidyltransferase activity, CDPdiacylglycerol-serine O-phosphatidyltransferase activity, CDPdiglyceride-serine O-phosphatidyltransferase activity, PS synthase activity, cytidine 5'-diphospho-1,2-diacyl-sn-glycerol (CDPdiglyceride):L-serine O-phosphatidyltransferase activity, cytidine 5'-diphospho-1,2-diacyl-sn-glycerol:L-serine O-phosphatidyltransferase activity, cytidine diphosphoglyceride-serine O-phosphatidyltransferase activity, phosphatidylserine synthase activity, phosphatidylserine synthetase activity